{
  "term_id": "UNKNOWN:0001",
  "term_label": "Unknown molecular function",
  "gene_symbol": "PSMD1",
  "gene_name": "26S proteasome non-ATPase regulatory subunit 1",
  "gene": "UniProtKB:Q99460"
}